{
  "term_label": "calcium-dependent protein serine/threonine phosphatase regulator activity",
  "gene": "UniProtKB:P63098",
  "term_id": "GO:0008597",
  "gene_symbol": "PPP3R1",
  "gene_name": "Calcineurin subunit B type 1"
}